{
  "gene_symbol": "B3GNT2",
  "gene_name": "N-acetyllactosaminide beta-1,3-N-acetylglucosaminyltransferase 2",
  "term_id": "GO:0008532",
  "gene": "UniProtKB:Q9NY97",
  "term_label": "N-acetyllactosaminide beta-1,3-N-acetylglucosaminyltransferase activity"
}